{
  "term_label": "positive regulation of cell migration",
  "term_id": "GO:0030335",
  "gene": "UniProtKB:O95025",
  "gene_name": "Semaphorin-3D",
  "gene_symbol": "SEMA3D"
}